aldaric acid catabolic process [GO:0019579] (biological process) Definition: The chemical reactions and pathways resulting in the breakdown of aldaric acid, any dicarboxylic acid formed by oxidation of by the terminal groups of an aldose to carboxyl group. Relationships: is_a dicarboxylic acid catabolic process [GO:0043649] Subtypes: glucarate catabolic process [GO:0019394], galactarate catabolic process [GO:0046392], L-altrarate catabolic process [GO:1903663] Sources: ISBN:0198506732 Also known as: aldaric acid breakdown, aldaric acid catabolism, aldaric acid degradation